GTPase activity [GO:0003924] (molecular function) Definition: Catalysis of the reaction: GTP + H2O = GDP + H+ + phosphate. Regulation: negatively regulated by GTPase inhibitor activity [GO:0005095]; positively regulated by GTPase activator activity [GO:0005096]; regulated by GTPase regulator activity [GO:0030695]; negatively regulated by negative regulation of GTPase activity [GO:0034260]; regulated by regulation of GTPase activity [GO:0043087]; positively regulated by positive regulation of GTPase activity [GO:0043547] Also known as: hydrolase activity, acting on acid anhydrides, acting on GTP, involved in cellular and subcellular movement, ARF small monomeric GTPase activity, RHEB small monomeric GTPase activity, Rab small monomeric GTPase activity, Ran small monomeric GTPase activity, Ras small monomeric GTPase activity, Rho small monomeric GTPase activity, Sar small monomeric GTPase activity, dynamin GTPase activity, heterotrimeric G-protein GTPase activity, protein-synthesizing GTPase activity, protein-synthesizing GTPase activity, elongation, protein-synthesizing GTPase activity, initiation, protein-synthesizing GTPase activity, termination, signal-recognition-particle GTPase activity, small monomeric GTPase activity, tubulin GTPase activity, GTPase activity, coupled, heterotrimeric G-protein GTPase, alpha-subunit, heterotrimeric G-protein GTPase, beta-subunit, heterotrimeric G-protein GTPase, gamma-subunit References: PMID:26832457, PMID:27218782 Subtypes: G protein activity [GO:0003925], GO:0061791, GTPase-dependent fusogenic activity [GO:0140523] Relationships: is a type of ribonucleoside triphosphate phosphatase activity [GO:0017111]